cranial nerve maturation [GO:0021605] (BP) Definition: A developmental process, independent of morphogenetic (shape) change, that is required for a cranial nerve to attain its fully functional state. The cranial nerves are composed of twelve pairs of nerves that emanate from the nervous tissue of the hindbrain. These nerves are sensory, motor, or mixed in nature, and provide the motor and general sensory innervation of the head, neck and viscera. They mediate vision, hearing, olfaction and taste and carry the parasympathetic innervation of the autonomic ganglia that control visceral functions. Sources: GOC:cls, GOC:dgh, GOC:dph, GOC:jid, GO_REF:0000021 Subtypes: abducens nerve maturation [GO:0021601], GO:0021606, facial nerve maturation [GO:0021613], glossopharyngeal nerve maturation [GO:0021614], hypoglossal nerve maturation [GO:0021619], oculomotor nerve maturation [GO:0021625], olfactory nerve maturation [GO:0021630], GO:0021632, trigeminal nerve maturation [GO:0021635], GO:0021640, vagus nerve maturation [GO:0021643], vestibulocochlear nerve maturation [GO:0021647] Relationships: is a type of nerve maturation [GO:0021682]; is part of cranial nerve development [GO:0021545]